regulation of cellular pH reduction [GO:0032847] (biological process) Subtypes: negative regulation of cellular pH reduction [GO:0032848], positive regulation of cellular pH reduction [GO:0032849], regulation of Golgi lumen acidification [GO:1905526] Definition: Any process that modulates the frequency, rate, or extent of a process that reduces the internal pH of a cell. Sources: GOC:mah Also known as: regulation of cell pH reduction, regulation of cellular acidification, regulation of intracellular pH reduction, regulation of reduction of cellular pH, regulation of reduction of pH in cell, regulation of intracellular acidification Relationships: is a type of regulation of biological process [GO:0050789]; is a type of regulation of intracellular pH [GO:0051453]; regulates GO:0051452